eukaryotic initiation factor 4E binding [GO:0008190] (molecular function) Definition: Binding to eukaryotic initiation factor 4E, a polypeptide factor involved in the initiation of ribosome-mediated translation. Sources: ISBN:0198506732 Relationships: is a type of translation initiation factor binding [GO:0031369] Also known as: eIF4E binding